syn-copalyl diphosphate synthase activity [GO:0051498] (MF) Sources: MetaCyc:RXN-8528 Definition: Catalysis of the reaction: geranylgeranyl diphosphate = 9alpha-copalyl diphosphate. Also known as: diterpene cyclase activity Relationships: is a type of GO:0016872